{
  "gene_name": "Transcription factor E2F1",
  "gene": "UniProtKB:Q01094",
  "term_label": "DNA-binding transcription factor activity, RNA polymerase II-specific",
  "term_id": "GO:0000981",
  "gene_symbol": "E2F1"
}